hepaticobiliary system process [GO:0061007] (BP) Definition: A system process carried out by any of the organs or tissues of the hepaticobiliary system. The hepaticobiliary system is responsible for metabolic and catabolic processing of small molecules absorbed from the blood or gut, hormones and serum proteins, detoxification, storage of glycogen, triglycerides, metals and lipid soluble vitamins and excretion of bile. Included are the synthesis of albumin, blood coagulation factors, complement, and specific binding proteins. Also known as: hepatobiliary system process Relationships: is a type of system process [GO:0003008] Sources: GOC:dph